{
  "gene": "UniProtKB:Q9NSB8",
  "gene_symbol": "HOMER2",
  "gene_name": "Homer protein homolog 2",
  "term_id": "GO:2001256",
  "term_label": "regulation of store-operated calcium entry"
}